positive regulation of smooth muscle cell migration [GO:0014911] (biological process) Sources: CL:0000192, GOC:mtg_muscle Subtypes: positive regulation of smooth muscle cell chemotaxis [GO:0071673], positive regulation of vascular associated smooth muscle cell migration [GO:1904754] Definition: Any process that activates, maintains or increases the frequency, rate or extent of smooth muscle cell migration. Relationships: is a type of regulation of smooth muscle cell migration [GO:0014910]; is a type of positive regulation of cell migration [GO:0030335]; positively regulates smooth muscle cell migration [GO:0014909]